{
  "term_id": "GO:0005525",
  "gene": "UniProtKB:Q15669",
  "gene_symbol": "RHOH",
  "gene_name": "Rho-related GTP-binding protein RhoH",
  "term_label": "GTP binding"
}